benzoyl-CoA 3-monooxygenase activity [GO:0047090] (molecular function) Relationships: is a type of oxidoreductase activity, acting on paired donors, with incorporation or reduction of molecular oxygen, NAD(P)H as one donor, and incorporation of one atom of oxygen [GO:0016709] Also known as: benzoyl-CoA 3-hydroxylase activity, benzoyl-CoA,NADPH:oxygen oxidoreductase (3-hydroxylating) Definition: Catalysis of the reaction: benzoyl-CoA + H+ + NADPH + O2 = 3-hydroxybenzoyl-CoA + H2O + NADP+. Sources: EC:1.14.13.58, RHEA:23216